reservosome [GO:0106123] (cellular component) Relationships: is_a storage vacuole [GO:0000322]; is a type of lytic vacuole [GO:0000323] References: PMID:12204365, PMID:15521631, PMID:1845219, PMID:19288526, PMID:21818313, PMID:22425988 Sources: GOC:ach Definition: A large membrane-bound endocytic organelle present only in members of the Schizotrypanum subgenus of the Trypanosoma genus and is defined as the site of storage of endocytosed macromolecules and lysosomal enzymes. It is found at the posterior end of epimastigote forms of Trypanosoma cruzi, but absent in amastigotes and trypomastigotes.